{
  "term_id": "GO:0006102",
  "term_label": "isocitrate metabolic process",
  "gene": "UniProtKB:O43837",
  "gene_name": "Isocitrate dehydrogenase [NAD] subunit beta, mitochondrial",
  "gene_symbol": "IDH3B"
}